{
  "term_id": "GO:1990430",
  "term_label": "extracellular matrix protein binding",
  "gene_symbol": "MEPE",
  "gene": "UniProtKB:Q9NQ76",
  "gene_name": "Matrix extracellular phosphoglycoprotein"
}